mitophagy by internal vacuole formation [GO:0035695] (biological process) Relationships: is a type of autophagy of mitochondrion [GO:0000422] Note: In this mechanism of mitochondrion degradation, the mitochondrion is directly engulfed by a lysosome-like vacuole. It is therefore distinct from canonical autophagy, which is mediated by a double-membrane autophagosome. References: PMID:21264228 Sources: GOC:autophagy, GOC:bf, GOC:sp Definition: The process in which cells degrade mitochondria by inducing a vacuole-like structure which directly engulfs and degrades the unhealthy mitochondria by accumulating lysosomes. Also known as: MIV-mediated mitophagy